{
  "term_label": "nucleus",
  "term_id": "GO:0005634",
  "gene_name": "Spermatogenic leucine zipper protein 1",
  "gene_symbol": "SPZ1",
  "gene": "UniProtKB:Q9BXG8"
}